{
  "gene_symbol": "SH2D3A",
  "gene": "UniProtKB:Q9BRG2",
  "term_label": "Unknown biological process",
  "term_id": "UNKNOWN:0002",
  "gene_name": "SH2 domain-containing protein 3A"
}